{
  "gene": "UniProtKB:Q2WGJ9",
  "term_label": "Unknown molecular function",
  "term_id": "UNKNOWN:0001",
  "gene_name": "Fer-1-like protein 6",
  "gene_symbol": "FER1L6"
}